glucosinolate biosynthetic process [GO:0019761] (biological process) Also known as: glucosinolate anabolism, glucosinolate biosynthesis, glucosinolate formation, glucosinolate synthesis Subtypes: indole glucosinolate biosynthetic process [GO:0009759], glucosinolate biosynthetic process from homomethionine [GO:0033506], glucosinolate biosynthetic process from phenylalanine [GO:0033507], 2-hydroxy-but-3-enyl glucosinolate biosynthetic process [GO:0080035] Relationships: is a type of S-glycoside biosynthetic process [GO:0016144]; is a type of glucosinolate metabolic process [GO:0019760] Definition: The chemical reactions and pathways resulting in the formation of glucosinolates, substituted thioglucosides found in rapeseed products and related cruciferae. Sources: GOC:ai Regulation: regulated by regulation of glucosinolate biosynthetic process [GO:0010439]